{
  "term_label": "polypeptide N-acetylgalactosaminyltransferase activity",
  "gene": "UniProtKB:Q8NCW6",
  "term_id": "GO:0004653",
  "gene_name": "Polypeptide N-acetylgalactosaminyltransferase 11",
  "gene_symbol": "GALNT11"
}